{
  "term_id": "GO:0001817",
  "gene_symbol": "ZBTB14",
  "term_label": "regulation of cytokine production",
  "gene_name": "Zinc finger and BTB domain-containing protein 14",
  "gene": "UniProtKB:O43829"
}